{
  "gene": "UniProtKB:Q9GZS9",
  "term_id": "GO:0018146",
  "term_label": "keratan sulfate proteoglycan biosynthetic process",
  "gene_name": "Carbohydrate sulfotransferase 5",
  "gene_symbol": "CHST5"
}